juxtaparanode region of axon [GO:0044224] (cellular component) Relationships: is a type of cellular anatomical structure [GO:0110165]; is part of main axon [GO:0044304] References: PMID:10624965, PMID:14682359 Sources: GOC:BHF, GOC:jl Also known as: juxtaparanodal region, juxtaparanode, juxta paranode axon Definition: A region of an axon near a node of Ranvier that is between the paranode and internode regions.